mesenchymal cell differentiation involved in mammary gland development [GO:0060610] (biological process) Also known as: mammary gland mesenchymal cell differentiation Sources: GOC:dph Relationships: is_a mesenchymal cell differentiation [GO:0048762]; is part of GO:0030879 Definition: The process in which a relatively unspecialized cell acquires specialized features of a mammary gland mesenchymal cell. Mammary gland mesenchymal cells form a loosely connected network of cells that surround the mammary ducts.